{
  "gene_name": "TBC1 domain family member 10A",
  "term_id": "UNKNOWN:0003",
  "gene": "UniProtKB:Q9BXI6",
  "gene_symbol": "TBC1D10A",
  "term_label": "Unknown cellular component"
}